{
  "term_id": "GO:0061631",
  "gene_name": "Ubiquitin-conjugating enzyme E2 R1",
  "gene": "UniProtKB:P49427",
  "term_label": "ubiquitin conjugating enzyme activity",
  "gene_symbol": "CDC34"
}